{
  "term_label": "basolateral plasma membrane",
  "gene": "UniProtKB:Q9NP59",
  "gene_symbol": "SLC40A1",
  "gene_name": "Solute carrier family 40 member 1",
  "term_id": "GO:0016323"
}